{
  "term_label": "Unknown cellular component",
  "gene_symbol": "CFAP52",
  "term_id": "UNKNOWN:0003",
  "gene_name": "Cilia- and flagella-associated protein 52",
  "gene": "UniProtKB:Q8N1V2"
}